{
  "gene_symbol": "ABTB1",
  "gene_name": "Ankyrin repeat and BTB_POZ domain-containing protein 1",
  "term_id": "GO:0005737",
  "term_label": "cytoplasm",
  "gene": "UniProtKB:Q969K4"
}